{
  "gene_symbol": "IRAK2",
  "gene_name": "Interleukin-1 receptor-associated kinase-like 2",
  "gene": "UniProtKB:O43187",
  "term_id": "GO:0005886",
  "term_label": "plasma membrane"
}